{
  "gene": "UniProtKB:Q13868",
  "term_id": "GO:0071034",
  "gene_name": "Exosome complex component RRP4",
  "gene_symbol": "EXOSC2",
  "term_label": "CUT catabolic process"
}